{
  "gene_name": "Double-strand break repair protein MRE11",
  "term_id": "GO:0030870",
  "term_label": "Mre11 complex",
  "gene_symbol": "MRE11",
  "gene": "UniProtKB:P49959"
}